myelination of posterior lateral line nerve axons [GO:0048932] (biological process) Definition: The formation of compact myelin sheaths around the axons of the posterior lateral line nerve. References: PMID:12112375 Relationships: is a type of myelination of lateral line nerve axons [GO:0048897]; is part of posterior lateral line nerve glial cell morphogenesis involved in differentiation [GO:0048942]